anthocyanin 6''-O-malonyltransferase activity [GO:0033809] (molecular function) Sources: RHEA:16025 Relationships: is a type of GO:0016747 Also known as: 3MaT, Dv3MaT, malonyl-CoA:anthocyanidin-3-O-beta-D-glucoside 6''-O-malonyltransferase activity, malonyl-coenzymeA:anthocyanidin-3-O-beta-D-glucoside 6''-O-malonyltransferase activity Definition: Catalysis of the reaction: malonyl-CoA + an anthocyanidin 3-O-beta-D-glucoside = CoA + an anthocyanidin 3-O-(6-O-malonyl-beta-D-glucoside).